{
  "term_id": "UNKNOWN:0003",
  "gene_symbol": "C1orf43",
  "gene": "UniProtKB:Q9BWL3",
  "term_label": "Unknown cellular component",
  "gene_name": "Protein C1orf43"
}